{
  "term_id": "UNKNOWN:0001",
  "gene_symbol": "CCDC51",
  "term_label": "Unknown molecular function",
  "gene": "UniProtKB:Q96ER9",
  "gene_name": "Mitochondrial potassium channel"
}